{
  "gene_symbol": "LEFTY1",
  "gene_name": "Left-right determination factor 1",
  "term_label": "BMP signaling pathway",
  "term_id": "GO:0030509",
  "gene": "UniProtKB:O75610"
}